{
  "term_label": "unfolded protein binding",
  "gene_symbol": "UGGT2",
  "term_id": "GO:0051082",
  "gene_name": "UDP-glucose:glycoprotein glucosyltransferase 2",
  "gene": "UniProtKB:Q9NYU1"
}